positive regulation of development of symbiont in host [GO:0044129] (BP) Definition: Any process in which the symbiont activates or maintains its progression from an initial condition to a later condition, within the cells or tissues of the host organism. The host is defined as the larger of the organisms involved in the symbiotic interaction. Sources: GOC:jl, GOC:pamgo_curators Note: This term partially replaces the obsolete term 'positive regulation of growth or development of symbiont in host ; GO:0033666'. See also 'positive regulation of growth of symbiont in host ; GO:0044128'. Relationships: is a type of regulation of development of symbiont in host [GO:0044127]; is a type of GO:0044149; positively regulates GO:0044114